{
  "term_label": "indoleamine 2,3-dioxygenase activity",
  "gene_name": "Indoleamine 2,3-dioxygenase 1",
  "gene_symbol": "IDO1",
  "gene": "UniProtKB:P14902",
  "term_id": "GO:0033754"
}